3',5'-cGMP-inhibited cyclic-nucleotide phosphodiesterase activity [GO:0004119] (molecular function) Note: cGMP-inhibited cyclic-nucleotide phosphodiesterase activity Definition: Catalysis of the reaction: nucleoside 3',5'-cyclic phosphate + H2O = nucleoside 5'-phosphate; catalytic activity is decreased in the presence of cGMP. Relationships: is a type of GO:0004114 References: PMID:35216259 Sources: GOC:mah